filtration diaphragm assembly [GO:0036058] (biological process) Subtypes: nephrocyte diaphragm assembly [GO:0036059], slit diaphragm assembly [GO:0036060] Relationships: is a type of cell-cell junction assembly [GO:0007043] References: PMID:18971929 Sources: GOC:mtg_kidney_jan10 Definition: The aggregation, arrangement and bonding together of a set of components to form a filtration diaphragm, a specialized cell-cell junction found between the cells of the excretory system, which provides a barrier for filtration of blood or hemolymph.